{
  "gene_name": "Thrombospondin type-1 domain-containing protein 4",
  "term_id": "UNKNOWN:0001",
  "gene_symbol": "THSD4",
  "term_label": "Unknown molecular function",
  "gene": "UniProtKB:Q6ZMP0"
}